alanine:sodium symporter activity [GO:0015655] (molecular function) Sources: GOC:ai Definition: Enables the transfer of a solute or solutes from one side of a membrane to the other according to the reaction: alanine(out) + Na+(out) = alanine(in) + Na+(in). Subtypes: L-asparagine:sodium symporter activity [GO:0140901], L-glutamine:sodium symporter activity [GO:0140902] Relationships: is a type of amino acid:sodium symporter activity [GO:0005283]; is a type of GO:0005343; is a type of GO:0022858 Also known as: sodium:alanine symporter activity